circadian regulation of systemic arterial blood pressure [GO:0003052] (BP) Sources: GOC:mtg_cardio, GOC:rl Subtypes: circadian regulation of systemic arterial blood pressure by the suprachiasmatic nucleus [GO:0003054] Relationships: is a type of regulation of systemic arterial blood pressure [GO:0003073]; is a type of circadian rhythm [GO:0007623] Definition: Any process in which an organism modulates its blood pressure at different values with a regularity of approximately 24 hours.